adhesion of symbiont to host cell surface via host membrane cholesterol [GO:0141026] (biological process) References: PMID:17557817, PMID:23239883 Relationships: is a type of adhesion of symbiont to host cell [GO:0044650] Definition: The attachment of a symbiont to its host by binding to cholesterol on the host cell surface. The host is defined as the larger of the organisms involved in a symbiotic interaction.